NK T cell differentiation [GO:0001865] (biological process) References: PMID:10704459 Sources: GOC:add, ISBN:0781735149 Relationships: is a type of alpha-beta T cell differentiation [GO:0046632] Also known as: NK T lymphocyte differentiation, NK T-cell differentiation, NK T-lymphocyte differentiation, NKT cell differentiation, NT cell differentiation, natural T cell differentiation, natural killer T cell differentiation, NK T cell development Definition: The process in which a precursor cell type acquires the specialized features of a NK T cell. Note: Note that NK T cells are a distinct lineage of T cells expressing natural killer cell markers and having T cell receptors characterized by the usage of a restricted repertoire of variable region gene segments. Note that immunologists typically use the word 'development' to refer to cells of B or T cell lineages undergoing the process that GO describes as 'cell differentiation'. Regulation: regulated by GO:0051136; negatively regulated by negative regulation of NK T cell differentiation [GO:0051137]; positively regulated by positive regulation of NK T cell differentiation [GO:0051138]